{
  "gene_name": "Heat shock factor protein 2",
  "term_label": "Unknown biological process",
  "gene_symbol": "HSF2",
  "term_id": "UNKNOWN:0002",
  "gene": "UniProtKB:Q03933"
}